negative regulation of connective tissue replacement involved in inflammatory response wound healing [GO:1904597] (biological process) Relationships: is a type of GO:1904596; is a type of negative regulation of connective tissue replacement [GO:1905204]; negatively regulates connective tissue replacement involved in inflammatory response wound healing [GO:0002248] References: PMID:18245812 Sources: GOC:TermGenie, GOC:krc, GO_REF:0000058 Definition: Any process that stops, prevents or reduces the frequency, rate or extent of wound healing connective tissue replacement, which may be replaced with fibrotic material, that occurs as part of an inflammatory response. Also known as: down regulation of connective tissue replacement involved in inflammatory response wound healing, down-regulation of connective tissue replacement involved in inflammatory response wound healing, downregulation of connective tissue replacement involved in inflammatory response wound healing, down regulation of fibrosis during inflammatory response, down-regulation of fibrosis during inflammatory response, downregulation of fibrosis during inflammatory response, inhibition of connective tissue replacement involved in inflammatory response wound healing, inhibition of fibrosis during inflammatory response, negative regulation of fibrosis during inflammatory response, down regulation of connective tissue replacement during inflammatory response, down-regulation of connective tissue replacement during inflammatory response, downregulation of connective tissue replacement during inflammatory response, inhibition of connective tissue replacement during inflammatory response, negative regulation of connective tissue replacement during inflammatory response